{
  "gene_name": "Inter-alpha-trypsin inhibitor heavy chain H6",
  "term_id": "UNKNOWN:0001",
  "gene_symbol": "ITIH6",
  "term_label": "Unknown molecular function",
  "gene": "UniProtKB:Q6UXX5"
}